{
  "gene_symbol": "EFCC1",
  "term_label": "Unknown cellular component",
  "gene_name": "EF-hand and coiled-coil domain-containing protein 1",
  "gene": "UniProtKB:Q9HA90",
  "term_id": "UNKNOWN:0003"
}